regulation of axon regeneration [GO:0048679] (biological process) Definition: Any process that modulates the frequency, rate or extent of axon regeneration. Relationships: is a type of regulation of response to external stimulus [GO:0032101]; is a type of GO:0070570; is a type of regulation of response to wounding [GO:1903034]; regulates GO:0031103 Sources: GOC:dgh, GOC:dph, GOC:jid, GOC:lm Subtypes: positive regulation of axon regeneration [GO:0048680], negative regulation of axon regeneration [GO:0048681], regulation of collateral sprouting of intact axon in response to injury [GO:0048683], regulation of optical nerve axon regeneration [GO:1905591]